{
  "gene_name": "Glypican-6",
  "term_label": "cell surface",
  "term_id": "GO:0009986",
  "gene_symbol": "GPC6",
  "gene": "UniProtKB:Q9Y625"
}